{
  "gene_symbol": "OR1J2",
  "gene": "UniProtKB:Q8NGS2",
  "term_label": "plasma membrane",
  "gene_name": "Olfactory receptor 1J2",
  "term_id": "GO:0005886"
}